{
  "term_id": "GO:0002143",
  "gene_name": "Cytoplasmic tRNA 2-thiolation protein 1",
  "gene_symbol": "CTU1",
  "term_label": "tRNA wobble position uridine thiolation",
  "gene": "UniProtKB:Q7Z7A3"
}